{
  "term_label": "E-box binding",
  "gene_name": "Class E basic helix-loop-helix protein 22",
  "gene": "UniProtKB:Q8NFJ8",
  "gene_symbol": "BHLHE22",
  "term_id": "GO:0070888"
}